sodium-independent thromboxane transport [GO:0071721] (biological process) Definition: The directed, sodium-independent, movement of thromboxanes into, out of or within a cell, or between cells, by means of some agent such as a transporter or pore. A thromboxane is any of a class of oxygenated oxane derivatives, originally derived from prostaglandin precursors in platelets, that stimulate aggregation of platelets and constriction of blood vessels. Relationships: is a type of thromboxane transport [GO:0071717]; is a type of sodium-independent icosanoid transport [GO:0071718] Sources: GOC:mah